tagatose kinase activity [GO:0050317] (molecular function) Relationships: is a type of GO:0016301; is a type of phosphotransferase activity, alcohol group as acceptor [GO:0016773] Sources: EC:2.7.1.101, RHEA:15513 Definition: Catalysis of the reaction: D-tagatose + ATP = D-tagatose 6-phosphate + ADP + 2 H+. Also known as: ATP:D-tagatose 6-phosphotransferase activity, D-tagatose 6-phosphate kinase activity, tagatose 6-phosphate kinase (phosphorylating)